Kv4.2-DPP6 channel complex [GO:0071200] (cellular component) Definition: A voltage-gated potassium channel complex that contains the peptidase-related protein DPP6 associated with the channel via interaction with the Kv alpha subunit 4.2. References: PMID:12575952, PMID:15911355 Also known as: Kv4.2-DPPX channel complex Relationships: is_a voltage-gated potassium channel complex [GO:0008076]